{
  "gene_symbol": "NSMCE2",
  "gene_name": "E3 SUMO-protein ligase NSE2",
  "term_id": "GO:0061665",
  "term_label": "SUMO ligase activity",
  "gene": "UniProtKB:Q96MF7"
}